iron ion transmembrane transporter inhibitor activity [GO:0097690] (molecular function) Relationships: is a type of transporter inhibitor activity [GO:0141110]; RO_0002212 iron ion transmembrane transporter activity [GO:0005381] References: PMID:15514116 Sources: GOC:BHF, GOC:kom Note: An example of this is human hepcidin (UniProt symbol P81172), which regulates iron transport out of cells (see PMID:15514116). Also known as: iron channel inhibitor activity Definition: Binds to and stops, prevents, or reduces the activity of an iron ion transmembrane transporter.